Isw1b complex [GO:0036437] (cellular component) Definition: An Isw1 complex that binds DNA and has nucleosome-stimulated ATPase activity. In S. cerevisiae, contains an Isw1p ATPase subunit in complex with Ioc2p and Ioc4p. References: PMID:12482963 Sources: GOC:jd Relationships: is a type of Isw1 complex [GO:0016587]